{
  "term_label": "oxidoreductase activity",
  "gene_name": "Lysine-specific histone demethylase 2",
  "gene_symbol": "KDM1B",
  "gene": "UniProtKB:Q8NB78",
  "term_id": "GO:0016491"
}